aorta smooth muscle tissue morphogenesis [GO:0060414] (biological process) Relationships: is a type of muscle tissue morphogenesis [GO:0060415]; is part of aorta morphogenesis [GO:0035909]; is part of GO:0048745 Sources: GOC:bf, GOC:dgh, GOC:dph, Wikipedia:Aorta Definition: The process in which the structure of the smooth muscle tissue surrounding the aorta is generated and organized. An aorta is an artery that carries blood from the heart to other parts of the body.